medium-chain fatty acid catabolic process [GO:0051793] (biological process) Note: While there is not universal consensus on the lengths of short-, medium-, long- and very-long-chain fatty acids, the GO uses the definitions in ChEBI (see CHEBI:26666, CHEBI:59554, CHEBI:15904 and CHEBI:27283). Relationships: is a type of fatty acid catabolic process [GO:0009062]; is a type of medium-chain fatty acid metabolic process [GO:0051791] Sources: Wikipedia:Fatty_acid_metabolism Also known as: medium chain fatty acid catabolic process, medium chain fatty acid catabolism, medium-chain fatty acid breakdown, medium-chain fatty acid catabolism, medium-chain fatty acid degradation Definition: The chemical reactions and pathways resulting in the breakdown of a medium-chain fatty acid. A medium-chain fatty acid has an aliphatic tail containing 6 to 12 carbons.